{
  "gene": "UniProtKB:Q969W1",
  "term_label": "palmitoyltransferase activity",
  "term_id": "GO:0016409",
  "gene_symbol": "ZDHHC16",
  "gene_name": "Palmitoyltransferase ZDHHC16"
}